cobalt ion transmembrane transporter activity [GO:0015087] (molecular function) Sources: GOC:dgf Also known as: cobalt, zinc uptake permease activity, zinc, cadmium, cobalt, nickel, lead-efflux ATPase activity Subtypes: P-type cobalt transporter activity [GO:0032778] Relationships: is a type of transition metal ion transmembrane transporter activity [GO:0046915]; is part of cobalt ion transport [GO:0006824] Definition: Enables the transfer of cobalt (Co2+) ions from one side of a membrane to the other.